glucose 1-dehydrogenase (NAD+) activity [GO:0047934] (molecular function) Definition: Catalysis of the reaction: D-glucose + NAD+ = D-glucono-1,5-lactone + NADH. Sources: EC:1.1.1.118, MetaCyc:GLUCOSE-1-DEHYDROGENASE-NAD+-RXN Also known as: D-aldohexose dehydrogenase activity, D-glucose:NAD oxidoreductase activity, D-glucose:NAD+ 1-oxidoreductase activity Relationships: is a type of glucose 1-dehydrogenase [NAD(P)+] activity [GO:0047936]